{
  "term_id": "UNKNOWN:0001",
  "term_label": "Unknown molecular function",
  "gene_symbol": "CBLN3",
  "gene": "UniProtKB:Q6UW01",
  "gene_name": "Cerebellin-3"
}